regulation of nuclear division [GO:0051783] (biological process) Subtypes: regulation of mitotic nuclear division [GO:0007088], regulation of meiotic nuclear division [GO:0040020], negative regulation of nuclear division [GO:0051784], positive regulation of nuclear division [GO:0051785] Relationships: is a type of regulation of organelle organization [GO:0033043]; regulates nuclear division [GO:0000280] Definition: Any process that modulates the frequency, rate or extent of nuclear division, the partitioning of the nucleus and its genetic information. Sources: GOC:ai